{
  "gene_symbol": "SETD3",
  "term_id": "GO:0018064",
  "gene_name": "Actin-histidine N-methyltransferase",
  "term_label": "protein-L-histidine N-tele-methyltransferase activity",
  "gene": "UniProtKB:Q86TU7"
}